{
  "gene": "UniProtKB:P06239",
  "term_id": "GO:0004715",
  "term_label": "non-membrane spanning protein tyrosine kinase activity",
  "gene_name": "Tyrosine-protein kinase Lck",
  "gene_symbol": "LCK"
}